{
  "gene_symbol": "SLC9A9",
  "term_id": "GO:0015385",
  "gene_name": "Sodium_hydrogen exchanger 9",
  "gene": "UniProtKB:Q8IVB4",
  "term_label": "sodium:proton antiporter activity"
}